{
  "gene": "UniProtKB:Q09028",
  "gene_name": "Histone-binding protein RBBP4",
  "gene_symbol": "RBBP4",
  "term_label": "ESC/E(Z) complex",
  "term_id": "GO:0035098"
}